{
  "term_label": "spliceosomal snRNP assembly",
  "gene": "UniProtKB:Q8WXD5",
  "term_id": "GO:0000387",
  "gene_name": "Gem-associated protein 6",
  "gene_symbol": "GEMIN6"
}